{
  "gene": "UniProtKB:Q96K17",
  "term_label": "Unknown biological process",
  "gene_name": "Transcription factor BTF3 homolog 4",
  "term_id": "UNKNOWN:0002",
  "gene_symbol": "BTF3L4"
}